{
  "term_label": "nuclear localization sequence binding",
  "term_id": "GO:0008139",
  "gene_symbol": "IPO4",
  "gene_name": "Importin-4",
  "gene": "UniProtKB:Q8TEX9"
}